{
  "gene_symbol": "LACC1",
  "term_id": "UNKNOWN:0002",
  "term_label": "Unknown biological process",
  "gene": "UniProtKB:Q8IV20",
  "gene_name": "Purine nucleoside phosphorylase LACC1"
}